presynaptic endocytosis [GO:0140238] (biological process) References: PMID:24719103 Note: Note that this term was created for the SynGO project, and will be obsoleted when the SynGO annotations are made in Noctua. Definition: A vesicle-mediated transport process in which the presynapse take up external materials or membrane constituents by the invagination of a small region of the plasma membrane to form a new membrane-bounded vesicle. Relationships: is a type of endocytosis [GO:0006897]; is_a establishment of localization in cell [GO:0051649]; is a type of vesicle-mediated transport in synapse [GO:0099003]; BFO_0000066 presynapse [GO:0098793] Subtypes: synaptic vesicle endocytosis [GO:0048488]